oxalate transmembrane transporter activity [GO:0019531] (molecular function) Definition: Enables the transfer of oxalate from one side of a membrane to the other. Oxalate, or ethanedioic acid, occurs in many plants and is highly toxic to animals. Sources: ISBN:0198506732 Also known as: oxalic acid transporter activity Relationships: is a type of dicarboxylic acid transmembrane transporter activity [GO:0005310]; is part of oxalate transport [GO:0019532] Subtypes: oxalate:chloride antiporter activity [GO:0160046]